{
  "gene": "UniProtKB:Q96L33",
  "term_id": "GO:0005886",
  "gene_symbol": "RHOV",
  "gene_name": "Rho-related GTP-binding protein RhoV",
  "term_label": "plasma membrane"
}